{
  "term_label": "AMPA glutamate receptor activity",
  "term_id": "GO:0004971",
  "gene_symbol": "GRIA1",
  "gene": "UniProtKB:P42261",
  "gene_name": "Glutamate receptor 1"
}